{
  "term_id": "UNKNOWN:0003",
  "gene": "UniProtKB:A6NM11",
  "gene_symbol": "LRRC37A2",
  "term_label": "Unknown cellular component",
  "gene_name": "Leucine-rich repeat-containing protein 37A2"
}